{
  "term_id": "UNKNOWN:0001",
  "gene_symbol": "LRRFIP2",
  "term_label": "Unknown molecular function",
  "gene_name": "Leucine-rich repeat flightless-interacting protein 2",
  "gene": "UniProtKB:Q9Y608"
}